{
  "term_label": "nucleus",
  "gene_name": "Friend leukemia integration 1 transcription factor",
  "term_id": "GO:0005634",
  "gene": "UniProtKB:Q01543",
  "gene_symbol": "FLI1"
}